response to inositol [GO:1902140] (biological process) References: PMID:16496115 Sources: GOC:TermGenie Relationships: is a type of response to oxygen-containing compound [GO:1901700] Subtypes: GO:1902141 Definition: Any process that results in a change in state or activity of a cell or an organism (in terms of movement, secretion, enzyme production, gene expression, etc.) as a result of an inositol stimulus.